2-oxoadipate reductase activity [GO:0047550] (molecular function) Relationships: is a type of oxidoreductase activity, acting on the CH-OH group of donors, NAD or NADP as acceptor [GO:0016616] Sources: EC:1.1.1.172, RHEA:14793 Also known as: 2-hydroxyadipate:NAD+ 2-oxidoreductase activity, 2-ketoadipate reductase activity, alpha-ketoadipate reductase activity Definition: Catalysis of the reaction: 2-hydroxyadipate + NAD+ = 2-oxoadipate + H+ + NADH.